{
  "gene": "UniProtKB:P35372",
  "gene_symbol": "OPRM1",
  "gene_name": "Mu-type opioid receptor",
  "term_id": "GO:0038003",
  "term_label": "G protein-coupled opioid receptor signaling pathway"
}